{
  "gene_symbol": "SLC47A2",
  "term_id": "UNKNOWN:0002",
  "gene": "UniProtKB:Q86VL8",
  "gene_name": "Multidrug and toxin extrusion protein 2",
  "term_label": "Unknown biological process"
}